monocoumaroyl dicaffeoyl spermidine meta-hydroxylase activity [GO:0072549] (molecular function) References: PMID:19779199 Sources: GOC:kad Definition: Catalysis of the reaction: monocoumaroyl dicaffeoyl spermidine + NADPH + O2 = tricaffeoyl spermidine + NADP+ + H2O. Relationships: is a type of tri-(coumaroyl or caffeoyl) spermidine meta-hydroxylase activity [GO:0072533]